V2 vasopressin receptor binding [GO:0031896] (molecular function) Relationships: is a type of vasopressin receptor binding [GO:0031893] Sources: GOC:mah, GOC:nln Also known as: V2 vasopressin receptor ligand Definition: Binding to a V2 vasopressin receptor.